{
  "gene_name": "Ragulator complex protein LAMTOR1",
  "gene": "UniProtKB:Q6IAA8",
  "term_label": "Ragulator complex",
  "gene_symbol": "LAMTOR1",
  "term_id": "GO:0071986"
}